{
  "term_label": "focal adhesion",
  "gene": "UniProtKB:Q68CZ2",
  "gene_name": "Tensin-3",
  "gene_symbol": "TNS3",
  "term_id": "GO:0005925"
}